{
  "gene": "UniProtKB:A1A5C7",
  "gene_symbol": "SLC22A23",
  "term_label": "Unknown molecular function",
  "term_id": "UNKNOWN:0001",
  "gene_name": "Solute carrier family 22 member 23"
}